{
  "gene_symbol": "PHKB",
  "term_id": "GO:0005964",
  "gene": "UniProtKB:Q93100",
  "gene_name": "Phosphorylase b kinase regulatory subunit beta",
  "term_label": "phosphorylase kinase complex"
}